{
  "gene": "UniProtKB:Q96QP1",
  "gene_symbol": "ALPK1",
  "gene_name": "Alpha-protein kinase 1",
  "term_id": "GO:0005929",
  "term_label": "cilium"
}